{
  "term_label": "Unknown cellular component",
  "gene_symbol": "SPATA31D3",
  "gene_name": "Spermatogenesis-associated protein 31D3",
  "term_id": "UNKNOWN:0003",
  "gene": "UniProtKB:P0C874"
}